{
  "gene_symbol": "DNAJC6",
  "term_label": "clathrin-dependent endocytosis",
  "gene": "UniProtKB:O75061",
  "gene_name": "Putative tyrosine-protein phosphatase auxilin",
  "term_id": "GO:0072583"
}